{
  "gene": "UniProtKB:P01860",
  "gene_name": "Immunoglobulin heavy constant gamma 3",
  "gene_symbol": "IGHG3",
  "term_label": "antibacterial humoral response",
  "term_id": "GO:0019731"
}